{
  "term_label": "tRNA binding",
  "gene_name": "RNA cytosine C(5)-methyltransferase NSUN2",
  "gene_symbol": "NSUN2",
  "gene": "UniProtKB:Q08J23",
  "term_id": "GO:0000049"
}